Kv4.3-DPP10 channel complex [GO:0071202] (cellular component) Also known as: Kv4.3-DPPY channel complex References: PMID:15911355 Relationships: is_a voltage-gated potassium channel complex [GO:0008076] Definition: A voltage-gated potassium channel complex that contains the peptidase-related protein DPP10 associated with the channel via interaction with the Kv alpha subunit 4.3.